{
  "gene_name": "Fragile X messenger ribonucleoprotein 1",
  "gene": "UniProtKB:Q06787",
  "term_id": "GO:0051028",
  "term_label": "mRNA transport",
  "gene_symbol": "FMR1"
}